{
  "term_id": "GO:0005794",
  "gene_symbol": "GRINA",
  "gene": "UniProtKB:Q7Z429",
  "term_label": "Golgi apparatus",
  "gene_name": "Protein lifeguard 1"
}